16-methoxy-2,3-dihydro-3-hydroxytabersonine N-methyltransferase activity [GO:0030768] (molecular function) Sources: EC:2.1.1.99, RHEA:11336 Also known as: 16-methoxy-2,3-dihydro-3-hydroxytabersonine methyltransferase activity, 3-hydroxy-16-methoxy-2,3-dihydrotabersonine N-methyltransferase activity, NMT activity, S-adenosyl-L-methionine:16-methoxy-2,3-dihydro-3-hydroxytabersonine N-methyltransferase activity, S-adenosyl-L-methionine:3-hydroxy-16-methoxy-2,3-dihydrotabersonine N-methyltransferase activity Relationships: is a type of S-adenosylmethionine-dependent methyltransferase activity [GO:0008757] Definition: Catalysis of the reaction: (3R)-3-hydroxy-16-methoxy-2,3-dihydrotabersonine + S-adenosyl-L-methionine = S-adenosyl-L-homocysteine + deacetoxyvindoline + H+.